{
  "term_id": "GO:0038036",
  "gene": "UniProtKB:P46089",
  "term_label": "sphingosine-1-phosphate receptor activity",
  "gene_name": "G-protein coupled receptor 3",
  "gene_symbol": "GPR3"
}